{
  "gene": "UniProtKB:P40429",
  "gene_symbol": "RPL13A",
  "term_id": "GO:0003735",
  "term_label": "structural constituent of ribosome",
  "gene_name": "Large ribosomal subunit protein uL13"
}